{
  "term_id": "GO:0016020",
  "gene_name": "Major facilitator superfamily domain-containing protein 3",
  "term_label": "membrane",
  "gene": "UniProtKB:Q96ES6",
  "gene_symbol": "MFSD3"
}